{
  "gene": "UniProtKB:Q7Z7L7",
  "term_label": "Cul2-RING ubiquitin ligase complex",
  "gene_symbol": "ZER1",
  "gene_name": "Protein zer-1 homolog",
  "term_id": "GO:0031462"
}